labyrinthine layer blood vessel development [GO:0060716] (biological process) Sources: GOC:dph Definition: The process whose specific outcome is the progression of a blood vessel of the labyrinthine layer of the placenta over time, from its formation to the mature structure. The embryonic vessels grow through the layer to come in close contact with the maternal blood supply. Relationships: is a type of GO:0048568; is a type of placenta blood vessel development [GO:0060674]; is part of labyrinthine layer development [GO:0060711]